{
  "term_label": "G protein-coupled neurotensin receptor activity",
  "gene_name": "Neurotensin receptor type 2",
  "term_id": "GO:0016492",
  "gene_symbol": "NTSR2",
  "gene": "UniProtKB:O95665"
}